{
  "gene_symbol": "CDC27",
  "term_id": "GO:0007091",
  "term_label": "metaphase/anaphase transition of mitotic cell cycle",
  "gene": "UniProtKB:P30260",
  "gene_name": "Cell division cycle protein 27 homolog"
}